(R)-4-hydroxyphenyllactate dehydrogenase (NADP+) activity [GO:0047029] (molecular function) Sources: RHEA:52692 Relationships: is a type of oxidoreductase activity, acting on the CH-OH group of donors, NAD or NADP as acceptor [GO:0016616] Definition: Catalysis of the reaction: NADP+ + (R)-3-(4-hydroxyphenyl)lactate = NADPH + H+ + 3-(4-hydroxyphenyl)pyruvate. Also known as: aromatic 2-oxoacid reductase activity, hydroxyphenylpyruvate reductase activity, phenylpyruvate reductase activity